{
  "gene_name": "Intermembrane lipid transfer protein VPS13A",
  "gene": "UniProtKB:Q96RL7",
  "term_label": "protein retention in Golgi apparatus",
  "term_id": "GO:0045053",
  "gene_symbol": "VPS13A"
}